resorcinol metabolic process [GO:0019505] (biological process) Also known as: 1,3-benzenediol metabolic process, 1,3-benzenediol metabolism, 1,3-dihydroxybenzene metabolic process, 1,3-dihydroxybenzene metabolism, resorcinol metabolism Definition: The chemical reactions and pathways involving resorcinol (C6H4(OH)2), a benzene derivative with many applications, including dyes, explosives, resins and as an antiseptic. References: PMID:33145, PMID:7217008 Sources: GOC:jl Relationships: is_a GO:0018958